{
  "gene_name": "AFG2-interacting ribosome maturation factor",
  "gene": "UniProtKB:Q9NX04",
  "term_id": "GO:0005634",
  "term_label": "nucleus",
  "gene_symbol": "AIRIM"
}